{
  "gene_symbol": "MUC22",
  "gene": "UniProtKB:E2RYF6",
  "term_id": "UNKNOWN:0002",
  "term_label": "Unknown biological process",
  "gene_name": "Mucin-22"
}